O-sinapoyltransferase activity [GO:0016753] (MF) Definition: Catalysis of the transfer of a sinapoyl group to an oxygen atom on the acceptor molecule. Subtypes: GO:0016754, sinapoylglucose-sinapoylglucose O-sinapoyltransferase activity [GO:0047158], sinapoylglucose-choline O-sinapoyltransferase activity [GO:0047202] Relationships: is a type of O-acyltransferase activity [GO:0008374]; is a type of sinapoyltransferase activity [GO:0016752] Sources: GOC:ai